positive regulation of MHC class I biosynthetic process [GO:0045345] (biological process) Sources: GOC:go_curators Definition: Any process that activates or increases the frequency, rate or extent of the chemical reactions and pathways resulting in the formation of MHC class I. Also known as: positive regulation of MHC class I anabolism, positive regulation of MHC class I biosynthesis, positive regulation of MHC class I formation, positive regulation of MHC class I synthesis, positive regulation of major histocompatibility complex class I biosynthesis, positive regulation of major histocompatibility complex class I biosynthetic process, up regulation of MHC class I biosynthetic process, up-regulation of MHC class I biosynthetic process, upregulation of MHC class I biosynthetic process, activation of MHC class I biosynthetic process, stimulation of MHC class I biosynthetic process Relationships: is a type of positive regulation of macromolecule biosynthetic process [GO:0010557]; is a type of regulation of MHC class I biosynthetic process [GO:0045343]; positively regulates MHC class I biosynthetic process [GO:0045341]